receptor internalization [GO:0031623] (biological process) Subtypes: G protein-coupled receptor internalization [GO:0002031], B cell receptor internalization [GO:0036300], regulation of signal transduction by receptor internalization [GO:0038009], insulin receptor internalization [GO:0038016], GO:0038017, neurotransmitter receptor internalization [GO:0099590] Regulation: regulated by regulation of receptor internalization [GO:0002090]; RO_0002212 by negative regulation of receptor internalization [GO:0002091]; positively regulated by GO:0002092 Definition: A receptor-mediated endocytosis process that results in the movement of receptors from the plasma membrane to the inside of the cell. The process begins when cell surface receptors are monoubiquitinated following ligand-induced activation. Receptors are subsequently taken up into endocytic vesicles from where they are either targeted to the lysosome or vacuole for degradation or recycled back to the plasma membrane. Relationships: is a type of receptor-mediated endocytosis [GO:0006898] References: PMID:15006537, PMID:19643732 Sources: GOC:bf, GOC:mah, GOC:signaling